{
  "gene_symbol": "CCK",
  "term_label": "extracellular space",
  "gene": "UniProtKB:P06307",
  "gene_name": "Cholecystokinin",
  "term_id": "GO:0005615"
}